{
  "gene_symbol": "CCND1",
  "term_id": "GO:0005634",
  "gene": "UniProtKB:P24385",
  "term_label": "nucleus",
  "gene_name": "G1_S-specific cyclin-D1"
}